{
  "gene": "UniProtKB:Q8IX07",
  "term_label": "nucleus",
  "gene_name": "Zinc finger protein ZFPM1",
  "gene_symbol": "ZFPM1",
  "term_id": "GO:0005634"
}